{
  "term_label": "NMDA glutamate receptor activity",
  "gene": "UniProtKB:Q14957",
  "term_id": "GO:0004972",
  "gene_symbol": "GRIN2C",
  "gene_name": "Glutamate receptor ionotropic, NMDA 2C"
}